{
  "term_id": "UNKNOWN:0001",
  "gene_symbol": "FAM169A",
  "gene_name": "Soluble lamin-associated protein of 75 kDa",
  "term_label": "Unknown molecular function",
  "gene": "UniProtKB:Q9Y6X4"
}